{
  "gene_name": "Mitogen-activated protein kinase 1",
  "term_label": "cell surface receptor signaling pathway",
  "term_id": "GO:0007166",
  "gene_symbol": "MAPK1",
  "gene": "UniProtKB:P28482"
}